{
  "term_id": "GO:0005886",
  "gene_symbol": "OR1D2",
  "term_label": "plasma membrane",
  "gene_name": "Olfactory receptor 1D2",
  "gene": "UniProtKB:P34982"
}